{
  "gene": "UniProtKB:Q96PU9",
  "gene_symbol": "CIMAP1A",
  "term_id": "GO:0001520",
  "term_label": "outer dense fiber",
  "gene_name": "Outer dense fiber protein 3"
}